{
  "gene_symbol": "MRPL49",
  "term_label": "Unknown biological process",
  "gene_name": "Large ribosomal subunit protein mL49",
  "term_id": "UNKNOWN:0002",
  "gene": "UniProtKB:Q13405"
}